{
  "term_id": "GO:0043005",
  "gene_name": "Neuronal acetylcholine receptor subunit alpha-3",
  "gene": "UniProtKB:P32297",
  "term_label": "neuron projection",
  "gene_symbol": "CHRNA3"
}